{
  "gene_symbol": "WEE2",
  "gene_name": "Wee1-like protein kinase 2",
  "term_label": "cytoplasm",
  "gene": "UniProtKB:P0C1S8",
  "term_id": "GO:0005737"
}